{
  "gene_symbol": "CCNL1",
  "gene_name": "Cyclin-L1",
  "gene": "UniProtKB:Q9UK58",
  "term_label": "nucleus",
  "term_id": "GO:0005634"
}